membrane depolarization during cardiac muscle cell action potential [GO:0086012] (biological process) Definition: The process in which cardiac muscle cell membrane potential changes in the depolarizing direction from the negative resting potential towards the positive membrane potential that will be the peak of the action potential. Sources: GOC:BHF, GOC:mtg_cardiac_conduct_nov11 Regulation: RO_0002211 by regulation of membrane depolarization during cardiac muscle cell action potential [GO:1900825]; negatively regulated by negative regulation of membrane depolarization during cardiac muscle cell action potential [GO:1900826]; positively regulated by positive regulation of membrane depolarization during cardiac muscle cell action potential [GO:1900827] Subtypes: membrane depolarization during AV node cell action potential [GO:0086045], membrane depolarization during SA node cell action potential [GO:0086046], GO:0086047, membrane depolarization during bundle of His cell action potential [GO:0086048], membrane depolarization during atrial cardiac muscle cell action potential [GO:0098912], membrane depolarization during ventricular cardiac muscle cell action potential [GO:0098913] Relationships: is a type of membrane depolarization during action potential [GO:0086010]; is part of GO:0086001